{
  "gene": "UniProtKB:Q7Z4S9",
  "term_id": "GO:0035556",
  "term_label": "intracellular signal transduction",
  "gene_symbol": "SH2D6",
  "gene_name": "SH2 domain-containing protein 6"
}